{
  "term_id": "UNKNOWN:0001",
  "gene_symbol": "TBATA",
  "gene_name": "Protein TBATA",
  "gene": "UniProtKB:Q96M53",
  "term_label": "Unknown molecular function"
}